{
  "gene_symbol": "PLXNA4",
  "gene_name": "Plexin-A4",
  "term_label": "synapse assembly",
  "term_id": "GO:0007416",
  "gene": "UniProtKB:Q9HCM2"
}